bacterial-type flagellum basal body, rod [GO:0030694] (cellular component) Also known as: flagellar basal body, rod, flagellin-based flagellum basal body, rod References: PMID:10572114, PMID:11133968, PMID:12624192 Sources: GOC:cilia, GOC:mtg_sensu Relationships: is a type of cellular anatomical structure [GO:0110165]; is part of GO:0009425 Definition: The central portion of the bacterial-type flagellar basal body, which spans the periplasm and threads through the rings.